inositol 1,4,5 trisphosphate binding [GO:0070679] (MF) Definition: Binding to inositol 1,4,5 trisphosphate. Sources: GOC:BHF, GOC:mah Also known as: IP3 binding, InsP3 binding Relationships: is a type of anion binding [GO:0043168]; is a type of GO:0043178